{
  "gene": "UniProtKB:Q8WWX0",
  "term_label": "protein ubiquitination",
  "gene_name": "Ankyrin repeat and SOCS box protein 5",
  "term_id": "GO:0016567",
  "gene_symbol": "ASB5"
}